{
  "gene": "UniProtKB:Q96MF7",
  "term_label": "double-strand break repair via homologous recombination",
  "term_id": "GO:0000724",
  "gene_symbol": "NSMCE2",
  "gene_name": "E3 SUMO-protein ligase NSE2"
}